regulation of plus-end directed microtubule sliding [GO:0062169] (biological process) Relationships: is a type of GO:0060632; regulates plus-end directed microtubule sliding [GO:0031535] Definition: Any process that mediates the frequency, rate, or extent of plus-end directed microtubule sliding. References: PMID:21892183 Subtypes: GO:0062168